{
  "gene_symbol": "FGFR2",
  "term_id": "GO:0008543",
  "term_label": "fibroblast growth factor receptor signaling pathway",
  "gene": "UniProtKB:P21802",
  "gene_name": "Fibroblast growth factor receptor 2"
}